{
  "gene": "UniProtKB:A0A1W2PRN1",
  "gene_symbol": "A0A1W2PRN1",
  "gene_name": "Golgin subfamily A conserved domain-containing protein",
  "term_label": "Unknown molecular function",
  "term_id": "UNKNOWN:0001"
}